transdifferentiation [GO:0060290] (biological process) Definition: The conversion of a differentiated cell of one fate into a differentiated cell of another fate without first undergoing cell division or reversion to a more primitive or stem cell-like fate. Sources: GOC:dph, GOC:kmv Regulation: regulated by regulation of transdifferentiation [GO:1903618]; negatively regulated by negative regulation of transdifferentiation [GO:1903619]; positively regulated by GO:1903620 Relationships: is a type of cell differentiation [GO:0030154]